virion transport vesicle [GO:0046816] (cellular component) Definition: A vesicle used to transport the partial or complete virion between cellular compartments. References: PMID:7933124 Sources: GOC:vesicles Relationships: is a type of intracellular vesicle [GO:0097708]